{
  "gene": "UniProtKB:Q9BYQ4",
  "term_id": "UNKNOWN:0001",
  "gene_symbol": "KRTAP9-2",
  "gene_name": "Keratin-associated protein 9-2",
  "term_label": "Unknown molecular function"
}